{
  "gene_symbol": "IGFBP4",
  "term_id": "GO:0043567",
  "gene_name": "Insulin-like growth factor-binding protein 4",
  "gene": "UniProtKB:P22692",
  "term_label": "regulation of insulin-like growth factor receptor signaling pathway"
}